{
  "term_label": "nucleus",
  "gene_symbol": "CDK11A",
  "gene_name": "Cyclin-dependent kinase 11A",
  "gene": "UniProtKB:Q9UQ88",
  "term_id": "GO:0005634"
}